endoplasmic reticulum palmitoyltransferase complex [GO:0031211] (cellular component) Relationships: is a type of GO:0002178; is a type of endoplasmic reticulum protein-containing complex [GO:0140534] Definition: A complex of the endoplasmic reticulum that catalyzes S-palmitoylation, the addition of palmitate (C16:0) or other long-chain fatty acids to proteins at a cysteine residue. Sources: GOC:jh